{
  "gene": "UniProtKB:A6NGC4",
  "term_label": "Unknown molecular function",
  "gene_symbol": "TLCD2",
  "term_id": "UNKNOWN:0001",
  "gene_name": "TLC domain-containing protein 2"
}